{
  "term_id": "UNKNOWN:0001",
  "gene_name": "Ataxin-7-like protein 1",
  "term_label": "Unknown molecular function",
  "gene_symbol": "ATXN7L1",
  "gene": "UniProtKB:Q9ULK2"
}